{
  "gene_symbol": "RAD23A",
  "gene": "UniProtKB:P54725",
  "term_label": "cytosol",
  "gene_name": "UV excision repair protein RAD23 homolog A",
  "term_id": "GO:0005829"
}